2,3-dihydroxybiphenyl 1,2-dioxygenase activity [GO:0043898] (molecular function) References: PMID:15715866 Sources: GOC:jl Definition: Catalysis of the reaction: 2,3-dihydroxybiphenyl + O2 = 2-hydroxy-6-phenylhexa-2,4-dienoic acid. Also known as: 2,3-dihydroxybiphenyl-1,2-dioxygenase activity, BphC Relationships: is a type of GO:0016702